{
  "gene": "UniProtKB:P08865",
  "term_label": "cytosolic small ribosomal subunit",
  "gene_name": "Small ribosomal subunit protein uS2",
  "gene_symbol": "RPSA",
  "term_id": "GO:0022627"
}